{
  "gene": "UniProtKB:Q8TF01",
  "term_id": "GO:0016607",
  "gene_symbol": "PNISR",
  "gene_name": "Arginine_serine-rich protein PNISR",
  "term_label": "nuclear speck"
}